{
  "gene_name": "Sulfhydryl oxidase 1",
  "gene": "UniProtKB:O00391",
  "gene_symbol": "QSOX1",
  "term_id": "GO:0016971",
  "term_label": "flavin-dependent sulfhydryl oxidase activity"
}